{
  "gene": "UniProtKB:Q4VX76",
  "term_id": "GO:0006887",
  "term_label": "exocytosis",
  "gene_symbol": "SYTL3",
  "gene_name": "Synaptotagmin-like protein 3"
}